{
  "gene_symbol": "FERMT3",
  "gene": "UniProtKB:Q86UX7",
  "gene_name": "Fermitin family homolog 3",
  "term_label": "integrin binding",
  "term_id": "GO:0005178"
}